Wnt signaling pathway, regulating spindle positioning [GO:0060069] (biological process) Definition: The series of molecular signals initiated by binding of Wnt protein to a frizzled family receptor on the surface of the target cell and ending with the positioning of the mitotic spindle. References: PMID:11532397 Sources: GOC:bf, GOC:dph Relationships: is a type of regulation of cell cycle process [GO:0010564]; is a type of regulation of localization [GO:0032879]; is_a GO:0035567; is a type of regulation of microtubule cytoskeleton organization [GO:0070507]; regulates establishment of mitotic spindle localization [GO:0040001] Also known as: non-canonical Wnt signaling pathway, Wnt receptor signaling pathway, regulating spindle positioning, Wnt receptor signalling pathway, regulating spindle positioning, Wnt-activated signaling pathway, regulating spindle positioning